{
  "gene_symbol": "ABHD16A",
  "gene": "UniProtKB:O95870",
  "gene_name": "Phosphatidylserine lipase ABHD16A",
  "term_label": "monoacylglycerol lipase activity",
  "term_id": "GO:0047372"
}